3,4-dichloroaniline N-malonyltransferase activity [GO:0047163] (molecular function) Relationships: is a type of N-malonyltransferase activity [GO:0050735] Also known as: malonyl-CoA:3,4-dichloroaniline N-malonyltransferase activity Sources: EC:2.3.1.114, RHEA:21060 Definition: Catalysis of the reaction: 3,4-dichloroaniline + malonyl-CoA = N-(3,4-dichlorophenyl)malonamate + CoA.